positive regulation of inositol trisphosphate biosynthetic process [GO:0032962] (biological process) Also known as: positive regulation of IP3 biosynthesis, positive regulation of IP3 biosynthetic process, positive regulation of inositol trisphosphate anabolism, positive regulation of inositol trisphosphate biosynthesis, positive regulation of inositol trisphosphate formation, positive regulation of inositol trisphosphate synthesis, positive regulation of myo-inositol trisphosphate biosynthesis, positive regulation of myo-inositol trisphosphate biosynthetic process Definition: Any process that activates or increases the frequency, rate or extent of the chemical reactions and pathways resulting in the formation of inositol trisphosphate. Sources: GOC:mah Relationships: is a type of GO:0032960; is a type of positive regulation of inositol phosphate biosynthetic process [GO:0060732]; positively regulates inositol trisphosphate biosynthetic process [GO:0032959]